{
  "term_id": "UNKNOWN:0002",
  "gene_name": "Uncharacterized protein ARIH2OS",
  "gene": "UniProtKB:Q8N7S6",
  "gene_symbol": "ARIH2OS",
  "term_label": "Unknown biological process"
}